{
  "term_id": "GO:0030425",
  "term_label": "dendrite",
  "gene_symbol": "HTR1A",
  "gene": "UniProtKB:P08908",
  "gene_name": "5-hydroxytryptamine receptor 1A"
}